cellular response to methionine [GO:0061431] (biological process) Relationships: is a type of GO:0031670; is a type of cellular response to amino acid stimulus [GO:0071230]; is a type of cellular response to nitrogen compound [GO:1901699]; is a type of GO:1901701; is a type of response to methionine [GO:1904640] Definition: Any process that results in a change in state or activity of a cell (in terms of movement, secretion, enzyme production, gene expression, etc.) as a result of a methionine stimulus. References: PMID:7891681 Sources: GOC:dph